{
  "gene_name": "Microtubule organization protein AKNA",
  "term_id": "GO:0021849",
  "gene": "UniProtKB:Q7Z591",
  "term_label": "neuroblast division in subventricular zone",
  "gene_symbol": "AKNA"
}